{
  "term_label": "Unknown cellular component",
  "gene": "UniProtKB:Q6ZPB5",
  "term_id": "UNKNOWN:0003",
  "gene_name": "Stress-responsive DNAJB4-interacting membrane protein 1",
  "gene_symbol": "SDIM1"
}